{
  "term_label": "proteasome-mediated ubiquitin-dependent protein catabolic process",
  "gene_name": "Kelch-like protein 35",
  "gene": "UniProtKB:Q6PF15",
  "term_id": "GO:0043161",
  "gene_symbol": "KLHL35"
}